negative regulation of antifungal innate immune response [GO:1905035] (biological process) Relationships: is a type of negative regulation of innate immune response [GO:0045824]; is a type of GO:1905034; negatively regulates GO:0061760 References: PMID:22470487 Sources: GOC:TermGenie, GOC:dph, GO_REF:0000058 Definition: Any process that stops, prevents or reduces the frequency, rate or extent of an antifungal innate immune response. Also known as: down regulation of antifungal innate immune response, down-regulation of antifungal innate immune response, downregulation of antifungal innate immune response, inhibition of antifungal innate immune response